{
  "term_label": "Unknown cellular component",
  "gene_name": "Putative protein BCL8",
  "gene": "UniProtKB:P0C6P0",
  "term_id": "UNKNOWN:0003",
  "gene_symbol": "NBEAP1"
}